metanephric interstitial fibroblast differentiation [GO:0072258] (biological process) Also known as: metanephros interstitial cell differentiation Definition: The process in which relatively unspecialized cells acquire specialized structural and/or functional features that characterize the interstitial fibroblasts of the metanephros as it progresses from its formation to the mature state. Sources: GOC:mtg_kidney_jan10 Relationships: is a type of kidney interstitial fibroblast differentiation [GO:0072071]; is a type of cell differentiation involved in metanephros development [GO:0072202]